{
  "gene_name": "Collagen alpha-1(XXV) chain",
  "term_id": "GO:0001540",
  "gene": "UniProtKB:Q9BXS0",
  "gene_symbol": "COL25A1",
  "term_label": "amyloid-beta binding"
}